regulation of T cell costimulation [GO:2000523] (biological process) Also known as: regulation of T cell co-stimulation, regulation of T lymphocyte costimulation, regulation of T-cell co-stimulation, regulation of T-cell costimulation, regulation of T-lymphocyte costimulation Definition: Any process that modulates the frequency, rate or extent of T cell costimulation. Subtypes: regulation of CD4-positive, alpha-beta T cell costimulation [GO:1900279], GO:2000524, positive regulation of T cell costimulation [GO:2000525] Sources: GOC:obol Relationships: is a type of GO:0050863; is a type of regulation of leukocyte cell-cell adhesion [GO:1903037]; regulates T cell costimulation [GO:0031295]